{
  "term_id": "GO:0003924",
  "gene_name": "Ras-related protein Rab-1B",
  "gene": "UniProtKB:Q9H0U4",
  "term_label": "GTPase activity",
  "gene_symbol": "RAB1B"
}